positive regulation of melanosome organization [GO:1903058] (biological process) References: PMID:24769727 Sources: GOC:BHF, GOC:TermGenie, GOC:rl, GO_REF:0000058 Note: Lack of the transcription factor Zeb2 Q9R0G7 leads to spherical melanosomes with irregular borders, in contrast to the rod-shaped melanosomes of ZEB2MCWT hair follicles. Relationships: is a type of positive regulation of organelle organization [GO:0010638]; is a type of regulation of melanosome organization [GO:1903056]; positively regulates melanosome organization [GO:0032438] Definition: Any process that activates or increases the frequency, rate or extent of melanosome organization. Also known as: positive regulation of melanosome organisation, up regulation of melanosome organisation, up regulation of melanosome organization, up-regulation of melanosome organisation, up-regulation of melanosome organization, upregulation of melanosome organisation, upregulation of melanosome organization, activation of melanosome organisation, activation of melanosome organization, activation of melanosome organization and biogenesis, positive regulation of melanosome organization and biogenesis, up regulation of melanosome organization and biogenesis, up-regulation of melanosome organization and biogenesis, upregulation of melanosome organization and biogenesis